flavonol biosynthetic process [GO:0051555] (biological process) Relationships: is a type of flavone biosynthetic process [GO:0051553]; is a type of flavonol metabolic process [GO:0051554] Definition: The chemical reactions and pathways resulting in the formation of flavonols, a member of a class of vascular pigments formed by consecutive oxidative processes from the flavonoid intermediates flavanones and dihydroflavonols. Flavonols are the most widespread of the flavonoids and have a wide array of physiological activities. Regulation: regulated by regulation of flavonol biosynthetic process [GO:1900384]; negatively regulated by negative regulation of flavonol biosynthetic process [GO:1900385]; positively regulated by positive regulation of flavonol biosynthetic process [GO:1900386] Sources: GOC:ai